{
  "term_id": "UNKNOWN:0001",
  "term_label": "Unknown molecular function",
  "gene": "UniProtKB:Q96DY2",
  "gene_symbol": "IQCD",
  "gene_name": "Dynein regulatory complex protein 10"
}